{
  "gene_symbol": "ST8SIA4",
  "gene": "UniProtKB:Q92187",
  "term_id": "GO:0009311",
  "gene_name": "CMP-N-acetylneuraminate-poly-alpha-2,8-sialyltransferase",
  "term_label": "oligosaccharide metabolic process"
}